{
  "gene_name": "Integrin beta-8",
  "gene_symbol": "ITGB8",
  "term_label": "cell adhesion mediated by integrin",
  "term_id": "GO:0033627",
  "gene": "UniProtKB:P26012"
}